{
  "gene_symbol": "KIF13A",
  "gene": "UniProtKB:Q9H1H9",
  "term_id": "GO:0005874",
  "gene_name": "Kinesin-like protein KIF13A",
  "term_label": "microtubule"
}